{
  "gene_symbol": "TMEM60",
  "term_label": "Unknown biological process",
  "term_id": "UNKNOWN:0002",
  "gene_name": "Transmembrane protein 60",
  "gene": "UniProtKB:Q9H2L4"
}